{
  "term_label": "immunoglobulin complex",
  "gene_name": "T cell receptor alpha variable 16",
  "gene": "UniProtKB:A0A0A6YYK6",
  "term_id": "GO:0019814",
  "gene_symbol": "TRAV16"
}